GMP catabolic process [GO:0046038] (biological process) Sources: GOC:go_curators Subtypes: GMP catabolic process to IMP [GO:0006201], GO:0006202 Also known as: GMP breakdown, GMP catabolism, GMP degradation Relationships: is a type of GO:0009154; is a type of purine ribonucleoside monophosphate catabolic process [GO:0009169]; is a type of GO:0046037 Definition: The chemical reactions and pathways resulting in the breakdown of GMP, guanosine monophosphate.